{
  "term_id": "GO:0000159",
  "gene": "UniProtKB:Q15173",
  "gene_symbol": "PPP2R5B",
  "gene_name": "Serine_threonine-protein phosphatase 2A 56 kDa regulatory subunit beta isoform",
  "term_label": "protein phosphatase type 2A complex"
}